nucleic acid metabolic process [GO:0090304] (biological process) Sources: GOC:dph, GOC:tb Note: This term should not be used for direct annotation. It should be possible to make a more specific annotation to one of the children of this term. Subtypes: GO:0006259, GO:0016070, nucleic acid biosynthetic process [GO:0141187], nucleic acid catabolic process [GO:0141188] Relationships: is a type of nucleobase-containing compound metabolic process [GO:0006139]; is a type of macromolecule metabolic process [GO:0043170] Definition: Any cellular metabolic process involving nucleic acids.